{
  "gene_symbol": "ARHGEF11",
  "gene": "UniProtKB:O15085",
  "term_label": "guanyl-nucleotide exchange factor activity",
  "gene_name": "Rho guanine nucleotide exchange factor 11",
  "term_id": "GO:0005085"
}